ribonuclease P4 activity [GO:0033894] (molecular function) Relationships: is a type of RNA endonuclease activity producing 5'-phosphomonoesters, hydrolytic mechanism [GO:0016891] Sources: EC:3.1.26.7 Definition: Catalysis of the endonucleolytic cleavage of RNA, removing 3'-extranucleotides from tRNA precursor.